activin receptor activity [GO:0017002] (molecular function) Definition: Combining with activin and transmitting the signal from one side of the membrane to the other to initiate a change in cell activity. Activin is one of two gonadal glycoproteins related to transforming growth factor beta. Sources: GOC:mah, GOC:signaling, ISBN:0198506732 Also known as: activin-activated receptor activity Note: Note that this term represents an activity and not a gene product, and should only be used when the receptor binds the ligand activin. For binding to other extracellular ligands, consider annotating to terms under 'transmembrane signaling receptor activity ; GO:0004888. Relationships: is_a transmembrane receptor protein serine/threonine kinase activity [GO:0004675]; is part of GO:0032924; has part activin binding [GO:0048185] Subtypes: activin receptor activity, type I [GO:0016361], GO:0016362